{
  "gene": "UniProtKB:O00469",
  "term_label": "collagen fibril organization",
  "gene_symbol": "PLOD2",
  "gene_name": "Procollagen-lysine,2-oxoglutarate 5-dioxygenase 2",
  "term_id": "GO:0030199"
}